{
  "term_id": "UNKNOWN:0001",
  "term_label": "Unknown molecular function",
  "gene_symbol": "ANKDD1A",
  "gene_name": "Ankyrin repeat and death domain-containing protein 1A",
  "gene": "UniProtKB:Q495B1"
}